{
  "term_label": "Unknown molecular function",
  "gene_symbol": "SIRPD",
  "term_id": "UNKNOWN:0001",
  "gene": "UniProtKB:Q9H106",
  "gene_name": "Signal-regulatory protein delta"
}